triferuloylspermidine meta-hydroxylase activity [GO:0072550] (molecular function) References: PMID:19779199 Sources: GOC:kad Also known as: triferuloyl spermidine meta-hydroxylase activity Relationships: is a type of tri-(feruloyl or hydroxyferuloyl) spermidine meta-hydroxylase activity [GO:0072532] Definition: Catalysis of the reaction: triferuloyl spermidine + NADPH + O2 = diferuloyl mono-(hydroxyferuloyl) spermidine + NADP+ + H2O.